bacterial degradosome [GO:1990061] (cellular component) Definition: The degradosome is a protein complex playing a key role in mRNA degradation and RNA processing. It includes a RNA helicase, a 3'-5' phosphate-dependent PNPase and a RNase E bound-enolase. Relationships: is a type of cytoplasmic exosome (RNase complex) [GO:0000177]; is part of GO:0005829 References: PMID:21805185 Sources: GOC:bhm